tRNA pseudouridine(38-40) synthase activity [GO:0160147] (molecular function) Definition: Catalysis of the reaction: uridine(38/39/40) in tRNA = pseudouridine(38/39/40) in tRNA. Relationships: is a type of tRNA pseudouridine synthase activity [GO:0106029] Sources: EC:5.4.99.12 Also known as: PSUI activity, tRNA pseudouridylate synthase